{
  "gene_symbol": "SF3B4",
  "gene": "UniProtKB:Q15427",
  "term_label": "mRNA splicing, via spliceosome",
  "gene_name": "Splicing factor 3B subunit 4",
  "term_id": "GO:0000398"
}